monoterpenyl-diphosphatase activity [GO:0050108] (molecular function) Also known as: monoterpenyl-pyrophosphatase activity, bornyl diphosphate hydrolase activity, bornyl pyrophosphate hydrolase activity, monoterpenyl-diphosphate diphosphohydrolase activity References: PMID:42357 Sources: EC:3.1.7.3 Relationships: is a type of phosphatase activity [GO:0016791] Definition: Catalysis of the reaction: (2S,4R)-bornyl diphosphate + H2O = (1R,2S,4R)-borneol + diphosphate.